{
  "gene_name": "Zinc finger protein 740",
  "term_label": "RNA polymerase II cis-regulatory region sequence-specific DNA binding",
  "gene": "UniProtKB:Q8NDX6",
  "term_id": "GO:0000978",
  "gene_symbol": "ZNF740"
}